{
  "gene_symbol": "PMFBP1",
  "term_label": "spermatogenesis",
  "term_id": "GO:0007283",
  "gene_name": "Polyamine-modulated factor 1-binding protein 1",
  "gene": "UniProtKB:Q8TBY8"
}